response to growth hormone-releasing hormone [GO:1990864] (biological process) Relationships: is a type of response to hormone [GO:0009725] Definition: Any process that results in a change in state or activity of a cell or an organism (in terms of movement, secretion, enzyme production, gene expression, etc.) as a result of a growth hormone-releasing hormone stimulus. Growth hormone-releasing hormone regulates the release of growth hormone, as well as some pancreatic proteins, and possibly other proteins. Also known as: response to GHRF, response to GRF, response to growth hormone-releasing factor, response to somatocrinin, response to somatoliberin, response to somatorelin, response to sermorelin References: PMID:7720628